{
  "gene_symbol": "OR2M5",
  "term_label": "detection of chemical stimulus involved in sensory perception of smell",
  "term_id": "GO:0050911",
  "gene_name": "Olfactory receptor 2M5",
  "gene": "UniProtKB:A3KFT3"
}